{
  "gene_name": "Methylcytosine dioxygenase TET3",
  "gene": "UniProtKB:O43151",
  "term_label": "DNA 5-methylcytosine dioxygenase activity",
  "term_id": "GO:0070579",
  "gene_symbol": "TET3"
}